{
  "gene": "UniProtKB:P62308",
  "term_id": "GO:0005682",
  "gene_symbol": "SNRPG",
  "gene_name": "Small nuclear ribonucleoprotein G",
  "term_label": "U5 snRNP"
}